{
  "gene_name": "Lipid transferase CIDEC",
  "term_id": "GO:0160077",
  "gene_symbol": "CIDEC",
  "gene": "UniProtKB:Q96AQ7",
  "term_label": "lipid droplet fusion"
}